{
  "gene_symbol": "BACE1",
  "term_label": "endosome",
  "gene_name": "Beta-secretase 1",
  "term_id": "GO:0005768",
  "gene": "UniProtKB:P56817"
}